{
  "term_id": "GO:0043066",
  "term_label": "negative regulation of apoptotic process",
  "gene": "UniProtKB:P26842",
  "gene_name": "CD27 antigen",
  "gene_symbol": "CD27"
}